{
  "term_id": "UNKNOWN:0003",
  "gene_name": "Glycerophosphocholine phosphodiesterase GPCPD1",
  "gene_symbol": "GPCPD1",
  "term_label": "Unknown cellular component",
  "gene": "UniProtKB:Q9NPB8"
}